intracellular potassium ion homeostasis [GO:0030007] (biological process) Also known as: cellular potassium ion homeostasis Relationships: is a type of intracellular monoatomic cation homeostasis [GO:0030003]; is a type of potassium ion homeostasis [GO:0055075] Sources: GOC:mah Definition: A homeostatic process involved in the maintenance of a steady state level of potassium ions within a cell.